{
  "gene_name": "Interleukin-9 receptor",
  "term_label": "immunoglobulin mediated immune response",
  "term_id": "GO:0016064",
  "gene": "UniProtKB:Q01113",
  "gene_symbol": "IL9R"
}